{
  "gene_name": "Hydroperoxide isomerase ALOXE3",
  "gene_symbol": "ALOXE3",
  "gene": "UniProtKB:Q9BYJ1",
  "term_label": "hepoxilin biosynthetic process",
  "term_id": "GO:0051122"
}